phosphomannomutase complex [GO:1990232] (cellular component) Also known as: PMM-1 complex, PMM-1 dimer, PMM-2 complex, PMM-2 dimer Relationships: is a type of intramolecular phosphotransferase complex [GO:1990233] References: PMID:16540464 Sources: GOC:bhm Definition: A protein complex capable of phosphomannomutase activity.